{
  "term_label": "Unknown molecular function",
  "term_id": "UNKNOWN:0001",
  "gene": "UniProtKB:Q9H069",
  "gene_symbol": "DRC3",
  "gene_name": "Dynein regulatory complex subunit 3"
}